{
  "gene_symbol": "SAXO2",
  "gene": "UniProtKB:Q658L1",
  "term_label": "microtubule binding",
  "gene_name": "Stabilizer of axonemal microtubules 2",
  "term_id": "GO:0008017"
}